response to ciliary neurotrophic factor [GO:1904391] (BP) References: PMID:16914133 Sources: GOC:TermGenie, GO_REF:0000071 Relationships: is a type of GO:1901698 Definition: Any process that results in a change in state or activity of a cell or an organism (in terms of movement, secretion, enzyme production, gene expression, etc.) as a result of a ciliary neurotrophic factor stimulus. Subtypes: GO:1904392